biphenyl synthase activity [GO:0033815] (molecular function) Sources: EC:2.3.1.177 Definition: Catalysis of the reaction: 3 malonyl-CoA + benzoyl-CoA = 4 CoA + 3,5-dihydroxybiphenyl + 4 CO2. Also known as: BIS, malonyl-CoA:benzoyl-CoA malonyltransferase activity Relationships: is a type of acyltransferase activity, transferring groups other than amino-acyl groups [GO:0016747]